type II polyketide synthase complex [GO:0034082] (cellular component) Definition: A polyketide synthase complex that consists of several different polypeptide chains, each of which catalyzes a single reaction. Relationships: is a type of polyketide synthase complex [GO:0034081] Also known as: type II PKS, type II PKS complex, type II polyketide synthase References: PMID:12636085 Sources: GOC:cb, GOC:mah